{
  "term_label": "intracellular protein transport",
  "term_id": "GO:0006886",
  "gene_name": "Syntaxin-4",
  "gene": "UniProtKB:Q12846",
  "gene_symbol": "STX4"
}